{
  "gene": "UniProtKB:P29122",
  "term_id": "GO:0031012",
  "term_label": "extracellular matrix",
  "gene_name": "Proprotein convertase subtilisin_kexin type 6",
  "gene_symbol": "PCSK6"
}